{
  "gene_name": "Zinc finger protein 665",
  "term_label": "RNA polymerase II cis-regulatory region sequence-specific DNA binding",
  "gene": "UniProtKB:Q9H7R5",
  "term_id": "GO:0000978",
  "gene_symbol": "ZNF665"
}